{
  "term_id": "GO:0005770",
  "gene_symbol": "CST7",
  "gene": "UniProtKB:O76096",
  "term_label": "late endosome",
  "gene_name": "Cystatin-F"
}